{
  "term_label": "Golgi cisterna membrane",
  "gene_symbol": "GOLGA8Q",
  "term_id": "GO:0032580",
  "gene": "UniProtKB:H3BV12",
  "gene_name": "Golgin subfamily A member 8Q"
}